{
  "term_id": "GO:0005634",
  "gene_name": "Proto-oncogene c-Rel",
  "gene_symbol": "REL",
  "gene": "UniProtKB:Q04864",
  "term_label": "nucleus"
}